fatty acid methyl ester biosynthetic process [GO:1902899] (biological process) Relationships: is a type of GO:1901570; is a type of GO:1902898 Definition: The chemical reactions and pathways resulting in the formation of fatty acid methyl ester. Also known as: FAME biosynthetic process, fatty acid methyl ester anabolism, fatty acid methyl ester biosynthesis, fatty acid methyl ester formation, fatty acid methyl ester synthesis References: PMID:16570218 Sources: GOC:TermGenie, GOC:mengo_curators, GO_REF:0000068